phosphate ion homeostasis [GO:0055062] (biological process) Also known as: phosphate homeostasis, Pi homeostasis Subtypes: intracellular phosphate ion homeostasis [GO:0030643] Sources: GOC:jid, GOC:mah Relationships: is a type of inorganic ion homeostasis [GO:0098771] Definition: Any process involved in the maintenance of an internal steady state of phosphate ions within an organism or cell.